channel activity [GO:0015267] (molecular function) Regulation: regulated by channel regulator activity [GO:0016247]; negatively regulated by GO:0016248; positively regulated by channel activator activity [GO:0099103] Definition: Enables the energy-independent facilitated diffusion of a solute through a transmembrane aqueous pore or channel. Stereospecificity is not exhibited but this transport may be specific for a particular molecular species or class of molecules. Subtypes: monoatomic ion channel activity [GO:0005216], GO:0008519, water channel activity [GO:0015250], glycerol channel activity [GO:0015254], methylammonium channel activity [GO:0015264], GO:0015265, wide pore channel activity [GO:0022829], gated channel activity [GO:0022836], GO:0022842, channel-forming ionophore activity [GO:0022886], GO:0140070, bicarbonate channel activity [GO:0160133], borate channel activity [GO:0180044] Sources: GOC:mtg_transport, ISBN:0815340729 Relationships: is a type of passive transmembrane transporter activity [GO:0022803] Also known as: pore activity, channel/pore class transporter activity, nonselective channel activity, alpha-type channel activity, channel-forming toxin activity, pore class transporter activity, substrate-specific channel activity